photoreceptor cell terminal bouton [GO:1990796] (cellular component) Definition: A specialized region of the axon terminus portion of a photoreceptor cell axon. A photoreceptor cell is a neuron specialized to detect and transduce light. Relationships: is a type of terminal bouton [GO:0043195] References: PMID:19883736